Malpighian tubule bud morphogenesis [GO:0061332] (biological process) Definition: The morphogenetic process in which a bud forms from the embryonic hindgut tube to form the Malpighian tubule. A bud is a protrusion that forms from the tube by localized changes in cell shape and position. References: PMID:19783135 Sources: GOC:dph, GOC:mtg_kidney_jan10 Relationships: is a type of morphogenesis of an epithelial bud [GO:0060572]; is a type of epithelial tube formation [GO:0072175]; is part of Malpighian tubule morphogenesis [GO:0007443] Also known as: Malpighian tubule formation